{
  "gene_name": "Forkhead box protein L3",
  "term_id": "GO:0009653",
  "gene": "UniProtKB:A0A1W2PRP0",
  "gene_symbol": "FOXL3",
  "term_label": "anatomical structure morphogenesis"
}